{
  "gene_symbol": "F11R",
  "gene_name": "Junctional adhesion molecule A",
  "gene": "UniProtKB:Q9Y624",
  "term_id": "GO:0090557",
  "term_label": "establishment of endothelial intestinal barrier"
}